{
  "gene_name": "Neuronal acetylcholine receptor subunit beta-2",
  "gene_symbol": "CHRNB2",
  "term_label": "monoatomic ion transmembrane transport",
  "gene": "UniProtKB:P17787",
  "term_id": "GO:0034220"
}